{
  "gene": "UniProtKB:P0C672",
  "term_label": "Unknown biological process",
  "gene_symbol": "TSPAN19",
  "gene_name": "Tetraspanin-19",
  "term_id": "UNKNOWN:0002"
}